{
  "term_id": "GO:0005829",
  "term_label": "cytosol",
  "gene_name": "Methionine--tRNA ligase, cytoplasmic",
  "gene": "UniProtKB:P56192",
  "gene_symbol": "MARS1"
}